thiamine-phosphate kinase activity [GO:0009030] (molecular function) Sources: EC:2.7.4.16, RHEA:15913 Definition: Catalysis of the reaction: ATP + thiamine phosphate = ADP + H+ + thiamine diphosphate. Relationships: is a type of kinase activity [GO:0016301]; is a type of phosphotransferase activity, phosphate group as acceptor [GO:0016776] Also known as: thiamin phosphate kinase activity, thiamin-phosphate kinase activity, ATP:thiamine-phosphate phosphotransferase activity, thiamin monophosphatase activity, thiamin monophosphokinase activity, thiamin-monophosphate kinase activity, thiamine-monophosphate kinase activity